{
  "gene_name": "Nucleotide-binding oligomerization domain-containing protein 1",
  "term_label": "intracellular signal transduction",
  "term_id": "GO:0035556",
  "gene": "UniProtKB:Q9Y239",
  "gene_symbol": "NOD1"
}